{
  "gene_name": "Centrosomal protein of 120 kDa",
  "gene_symbol": "CEP120",
  "term_id": "GO:1903724",
  "term_label": "positive regulation of centriole elongation",
  "gene": "UniProtKB:Q8N960"
}